{
  "gene_symbol": "NKG7",
  "gene": "UniProtKB:Q16617",
  "term_id": "UNKNOWN:0002",
  "term_label": "Unknown biological process",
  "gene_name": "Protein NKG7"
}